protein modification process [GO:0036211] (biological process) Subtypes: protein phosphorylation [GO:0006468], protein dephosphorylation [GO:0006470], protein sulfation [GO:0006477], protein lipidation [GO:0006497], protein deglycosylation [GO:0006517], protein alkylation [GO:0008213], GO:0008214, GO:0010731, protein arginylation [GO:0016598], protein flavinylation [GO:0017013], protein nitrosylation [GO:0017014], protein hydroxylation [GO:0018126], nucleic acid-protein covalent cross-linking [GO:0018143], GO:0018149, protein oxidation [GO:0018158], protein nucleotidylation [GO:0018175], protein polyamination [GO:0018184], peptidyl-amino acid modification [GO:0018193], GO:0018214, protein phosphopantetheinylation [GO:0018215], protein-coenzyme A linkage [GO:0018246], GO:0018249, GO:0018277, GO:0018282, protein-FAD linkage [GO:0018293], GO:0018342, protein-pyridoxal-5-phosphate linkage [GO:0018352], GO:0030047, N-terminal protein amino acid modification [GO:0031365], protein deacylation [GO:0035601], protein deglycation [GO:0036525], GO:0042040, protein acylation [GO:0043543], post-translational protein modification [GO:0043687], protein sulfhydration [GO:0044524], GO:0044601, protein carbamoylation [GO:0046944], protein delipidation [GO:0051697], protein de-ADP-ribosylation [GO:0051725], protein deglutathionylation [GO:0080058], protein sialylation [GO:1990743] Relationships: is a type of GO:0019538; is a type of macromolecule modification [GO:0043412] Also known as: cellular protein modification process, process resulting in protein modification, protein modification Regulation: regulated by regulation of protein modification process [GO:0031399]; RO_0002212 by GO:0031400; positively regulated by GO:0031401 Sources: GOC:bf, GOC:jl Definition: The covalent alteration of one or more amino acids occurring in proteins, peptides and nascent polypeptides (co-translational, post-translational modifications). Includes the modification of charged tRNAs that are destined to occur in a protein (pre-translation modification).